{
  "gene_name": "Leucine-rich repeat-containing protein 52",
  "term_label": "Unknown biological process",
  "gene_symbol": "LRRC52",
  "term_id": "UNKNOWN:0002",
  "gene": "UniProtKB:Q8N7C0"
}